{
  "term_label": "plasma membrane",
  "term_id": "GO:0005886",
  "gene": "UniProtKB:P34810",
  "gene_name": "Macrosialin",
  "gene_symbol": "CD68"
}